{
  "gene_symbol": "HLA-G",
  "gene": "UniProtKB:P17693",
  "term_label": "peptide antigen binding",
  "gene_name": "HLA class I histocompatibility antigen, alpha chain G",
  "term_id": "GO:0042605"
}